{
  "gene_symbol": "RBSN",
  "gene_name": "Rabenosyn-5",
  "gene": "UniProtKB:Q9H1K0",
  "term_id": "UNKNOWN:0003",
  "term_label": "Unknown cellular component"
}